sulfate transmembrane transport [GO:1902358] (biological process) Also known as: sulphate transport Definition: The directed movement of sulfate across a membrane. References: PMID:9055073 Sources: GOC:TermGenie, GOC:dph Relationships: is a type of inorganic anion transport [GO:0015698]; is a type of GO:0055085; is a type of GO:0072348 Subtypes: GO:1902434, mitochondrial sulfate transmembrane transport [GO:1990557]